{
  "gene_name": "Attractin-like protein 1",
  "term_id": "UNKNOWN:0003",
  "gene": "UniProtKB:Q5VV63",
  "gene_symbol": "ATRNL1",
  "term_label": "Unknown cellular component"
}